glycolate metabolic process [GO:0009441] (biological process) Definition: The chemical reactions and pathways involving glycolate, the anion of hydroxyethanoic acid (glycolic acid). Sources: GOC:ai, ISBN:0198506732 Also known as: glycolate metabolism Relationships: is a type of GO:0032787; is a type of primary alcohol metabolic process [GO:0034308] Subtypes: GO:0046295, GO:0046296